{
  "gene_name": "Deleted in malignant brain tumors 1 protein",
  "term_label": "scavenger receptor activity",
  "gene": "UniProtKB:Q9UGM3",
  "term_id": "GO:0005044",
  "gene_symbol": "DMBT1"
}